{
  "term_id": "GO:0000776",
  "gene_symbol": "AURKC",
  "gene": "UniProtKB:Q9UQB9",
  "gene_name": "Aurora kinase C",
  "term_label": "kinetochore"
}